{
  "gene": "UniProtKB:Q9NTX7",
  "gene_name": "E3 ubiquitin-protein ligase RNF146",
  "term_label": "cytoplasm",
  "term_id": "GO:0005737",
  "gene_symbol": "RNF146"
}